interleukin-5 receptor complex [GO:0005895] (cellular component) Also known as: IL-5 receptor complex References: PMID:11312115, PMID:11839579 Sources: GOC:mah Definition: A protein complex that binds interleukin-3; comprises an alpha and a beta subunit. The alpha chain is specific to the interleukin-5 receptor, whereas the beta chain is shared with the receptors for granulocyte-macrophage colony-stimulating factor and interleukin-3. Relationships: is a type of plasma membrane signaling receptor complex [GO:0098802]